{
  "term_label": "extracellular matrix",
  "gene_symbol": "TNXB",
  "term_id": "GO:0031012",
  "gene": "UniProtKB:P22105",
  "gene_name": "Tenascin-X"
}